{
  "term_label": "isocitrate dehydrogenase (NAD+) activity",
  "term_id": "GO:0004449",
  "gene": "UniProtKB:P50213",
  "gene_name": "Isocitrate dehydrogenase [NAD] subunit alpha, mitochondrial",
  "gene_symbol": "IDH3A"
}